{
  "gene_name": "Cell division cycle and apoptosis regulator protein 1",
  "term_id": "GO:0005634",
  "term_label": "nucleus",
  "gene": "UniProtKB:Q8IX12",
  "gene_symbol": "CCAR1"
}